{
  "gene_symbol": "FAM200B",
  "gene_name": "Protein FAM200B",
  "gene": "UniProtKB:P0CF97",
  "term_label": "Unknown cellular component",
  "term_id": "UNKNOWN:0003"
}